3-dehydro-L-gulonate-6-phosphate decarboxylase activity [GO:0033982] (molecular function) Definition: Catalysis of the reaction: 3-dehydro-L-gulonate 6-phosphate + H+ = L-xylulose 5-phosphate + CO2. Sources: EC:4.1.1.85, RHEA:14353 Relationships: is a type of carboxy-lyase activity [GO:0016831] Also known as: 3-dehydro-L-gulonate-6-phosphate carboxy-lyase (L-xylulose-5-phosphate-forming) activity, 3-dehydro-L-gulonate-6-phosphate carboxy-lyase activity, 3-keto-L-gulonate 6-phosphate decarboxylase activity, KGPDC, SgaH, SgbH, UlaD